{
  "gene_name": "Mitogen-activated protein kinase 14",
  "gene": "UniProtKB:Q16539",
  "term_label": "intracellular signal transduction",
  "gene_symbol": "MAPK14",
  "term_id": "GO:0035556"
}